{
  "term_id": "UNKNOWN:0002",
  "gene_name": "Arrestin domain-containing protein 5",
  "term_label": "Unknown biological process",
  "gene": "UniProtKB:A6NEK1",
  "gene_symbol": "ARRDC5"
}